{
  "term_id": "GO:0051082",
  "gene": "UniProtKB:P07900",
  "gene_symbol": "HSP90AA1",
  "term_label": "unfolded protein binding",
  "gene_name": "Heat shock protein HSP 90-alpha"
}